{
  "gene": "UniProtKB:A0A0C4DH39",
  "gene_symbol": "IGHV1-58",
  "gene_name": "Immunoglobulin heavy variable 1-58",
  "term_id": "GO:0003823",
  "term_label": "antigen binding"
}